{
  "gene_symbol": "RIN1",
  "term_label": "endocytic vesicle",
  "term_id": "GO:0030139",
  "gene_name": "Ras and Rab interactor 1",
  "gene": "UniProtKB:Q13671"
}